{
  "term_id": "GO:0030154",
  "gene_name": "Pro-neuregulin-1, membrane-bound isoform",
  "gene_symbol": "NRG1",
  "term_label": "cell differentiation",
  "gene": "UniProtKB:Q02297"
}